{
  "gene": "UniProtKB:P49281",
  "gene_symbol": "SLC11A2",
  "gene_name": "Natural resistance-associated macrophage protein 2",
  "term_id": "GO:0005384",
  "term_label": "manganese ion transmembrane transporter activity"
}